eye pigment catabolic process [GO:0046151] (biological process) Relationships: is a type of GO:0042441; is a type of pigment catabolic process [GO:0046149] Also known as: eye pigment breakdown, eye pigment catabolism, eye pigment degradation Sources: GOC:ai Definition: The chemical reactions and pathways resulting in the breakdown of eye pigments, any general or particular coloring matter in living organisms, found or utilized in the eye. Subtypes: ommochrome catabolic process [GO:0046153], rhodopsin catabolic process [GO:0046155]